G0 to G1 transition [GO:0045023] (biological process) Sources: GOC:mtg_cell_cycle, ISBN:0716731363 Definition: The mitotic cell cycle phase transition whose occurrence commits the cell from the G0 quiescent state to the G1 phase. Under certain conditions, cells exit the cell cycle during G1 and remain in the G0 state as nongrowing, non-dividing (quiescent) cells. Appropriate stimulation of such cells induces them to return to G1 and resume growth and division. The G0 to G1 transition is accompanied by many changes in the program of gene expression. Regulation: regulated by regulation of G0 to G1 transition [GO:0070316]; negatively regulated by negative regulation of G0 to G1 transition [GO:0070317]; positively regulated by positive regulation of G0 to G1 transition [GO:0070318] Relationships: is a type of GO:0022402